regulation of T cell mediated immune response to tumor cell [GO:0002840] (biological process) Sources: GOC:add Subtypes: negative regulation of T cell mediated immune response to tumor cell [GO:0002841], positive regulation of T cell mediated immune response to tumor cell [GO:0002842], regulation of T cell tolerance induction to tumor cell [GO:0002846], regulation of T cell mediated cytotoxicity directed against tumor cell target [GO:0002852] Definition: Any process that modulates the frequency, rate, or extent of a T cell mediated immune response to tumor cell. Also known as: regulation of T cell mediated immune response to tumour cell, regulation of T lymphocyte mediated immune response to tumor cell, regulation of T-cell mediated immune response to tumor cell, regulation of T-lymphocyte mediated immune response to tumor cell Relationships: is_a regulation of T cell mediated immunity [GO:0002709]; is a type of GO:0002837; regulates T cell mediated immune response to tumor cell [GO:0002424]